{
  "gene_name": "A disintegrin and metalloproteinase with thrombospondin motifs 12",
  "term_id": "GO:0004222",
  "gene": "UniProtKB:P58397",
  "term_label": "metalloendopeptidase activity",
  "gene_symbol": "ADAMTS12"
}